{
  "gene_name": "Keratin-associated protein 12-1",
  "gene_symbol": "KRTAP12-1",
  "gene": "UniProtKB:P59990",
  "term_label": "Unknown molecular function",
  "term_id": "UNKNOWN:0001"
}